{
  "gene": "UniProtKB:Q96NX5",
  "term_id": "GO:0004683",
  "term_label": "calcium/calmodulin-dependent protein kinase activity",
  "gene_symbol": "CAMK1G",
  "gene_name": "Calcium_calmodulin-dependent protein kinase type 1G"
}